{
  "gene_symbol": "CD72",
  "term_label": "Unknown molecular function",
  "gene_name": "B-cell differentiation antigen CD72",
  "term_id": "UNKNOWN:0001",
  "gene": "UniProtKB:P21854"
}